{
  "gene": "UniProtKB:O43541",
  "term_id": "GO:0006357",
  "term_label": "regulation of transcription by RNA polymerase II",
  "gene_symbol": "SMAD6",
  "gene_name": "Mothers against decapentaplegic homolog 6"
}